bradykinin catabolic process [GO:0010815] (biological process) Sources: GOC:BHF, GOC:rl Relationships: is a type of catabolic process [GO:0009056]; is a type of GO:0043603 Definition: The chemical reactions and pathways resulting in the breakdown of the peptide bradykinin.